aldonic acid biosynthetic process [GO:0046175] (biological process) Sources: ISBN:0198506732 Definition: The chemical reactions and pathways resulting in the formation of aldonic acid, a monocarboxylic acid with a chain of three or more carbon atoms, derived from an aldose by oxidation of the aldehydic group. Relationships: is a type of monocarboxylic acid biosynthetic process [GO:0072330] Subtypes: D-gluconate biosynthetic process [GO:0046178], GO:0046180, L-idonate biosynthetic process [GO:0046182] Also known as: aldonic acid anabolism, aldonic acid biosynthesis, aldonic acid formation, aldonic acid synthesis